{
  "term_id": "UNKNOWN:0002",
  "gene_symbol": "PYDC5",
  "gene_name": "Pyrin domain-containing protein 5",
  "term_label": "Unknown biological process",
  "gene": "UniProtKB:W6CW81"
}